{
  "term_id": "UNKNOWN:0003",
  "gene": "UniProtKB:Q6ISU1",
  "term_label": "Unknown cellular component",
  "gene_name": "Pre T-cell antigen receptor alpha",
  "gene_symbol": "PTCRA"
}